{
  "gene_name": "Neugrin",
  "term_label": "Unknown biological process",
  "gene": "UniProtKB:Q9NPE2",
  "gene_symbol": "NGRN",
  "term_id": "UNKNOWN:0002"
}